{
  "gene": "UniProtKB:Q08ER8",
  "term_id": "GO:0000981",
  "gene_name": "Zinc finger protein 543",
  "term_label": "DNA-binding transcription factor activity, RNA polymerase II-specific",
  "gene_symbol": "ZNF543"
}